{
  "term_id": "GO:0000132",
  "gene": "UniProtKB:Q86YR5",
  "gene_symbol": "GPSM1",
  "term_label": "establishment of mitotic spindle orientation",
  "gene_name": "G-protein-signaling modulator 1"
}